positive regulation of heart rate [GO:0010460] (biological process) Definition: Any process that activates or increases the frequency or rate of heart contraction. Sources: GOC:dph, GOC:tb Relationships: is a type of regulation of heart rate [GO:0002027]; is a type of positive regulation of heart contraction [GO:0045823] Subtypes: positive regulation of heart rate involved in baroreceptor response to decreased systemic arterial blood pressure [GO:0001988], GO:0001996, positive regulation of heart rate by epinephrine [GO:0003065], positive regulation of heart rate by norepinephrine [GO:0003066]